{
  "term_label": "peptide catabolic process",
  "gene": "UniProtKB:Q9NZ08",
  "gene_symbol": "ERAP1",
  "term_id": "GO:0043171",
  "gene_name": "Endoplasmic reticulum aminopeptidase 1"
}